{
  "term_id": "GO:0020037",
  "gene_symbol": "HBA2",
  "gene_name": "Hemoglobin subunit alpha",
  "gene": "UniProtKB:P69905",
  "term_label": "heme binding"
}